{
  "gene_name": "Liprin-alpha-3",
  "term_id": "GO:0048786",
  "term_label": "presynaptic active zone",
  "gene_symbol": "PPFIA3",
  "gene": "UniProtKB:O75145"
}